protein acetyltransferase complex [GO:0031248] (cellular component) Definition: A complex that catalyzes the transfer of an acetyl group to a protein acceptor molecule. Sources: GOC:bf Subtypes: histone acetyltransferase complex [GO:0000123], GO:0031414, NAGS/NAGK complex [GO:0106098] Relationships: is a type of intracellular protein-containing complex [GO:0140535]; is a type of GO:1902493